{
  "gene_symbol": "ANAPC7",
  "gene": "UniProtKB:Q9UJX3",
  "gene_name": "Anaphase-promoting complex subunit 7",
  "term_id": "GO:0016567",
  "term_label": "protein ubiquitination"
}